levansucrase activity [GO:0050053] (molecular function) Definition: Catalysis of the reaction: sucrose + 2,6-beta-D-fructosyl(n) = glucose + 2,6-beta-D-fructosyl(n+1). Relationships: is_a hexosyltransferase activity [GO:0016758] Also known as: beta-2,6-fructan:D-glucose 1-fructosyltransferase activity, beta-2,6-fructosyltransferase activity, sucrose 6-fructosyl transferase activity, sucrose 6-fructosyltransferase activity, sucrose:2,6-beta-D-fructan 6-beta-D-fructosyltransferase activity Sources: EC:2.4.1.10, MetaCyc:LEVANSUCRASE-RXN